{
  "gene_name": "G-protein coupled receptor family C group 5 member C",
  "gene": "UniProtKB:Q9NQ84",
  "term_label": "protein kinase activator activity",
  "term_id": "GO:0030295",
  "gene_symbol": "GPRC5C"
}